ligand-gated monoatomic anion channel activity [GO:0099095] (MF) Definition: Enables the transmembrane transfer of an inorganic anion by a channel that opens when a specific ligand has been bound by the channel complex or one of its constituent parts. Also known as: ligand-gated anion channel activity Subtypes: intracellularly calcium-gated chloride channel activity [GO:0005229], intracellularly ATP-gated chloride channel activity [GO:0005260], extracellularly glutamate-gated chloride channel activity [GO:0008068], extracellularly glycine-gated chloride channel activity [GO:0016934], GABA-gated chloride ion channel activity [GO:0022851], glycine-gated chloride ion channel activity [GO:0022852], pH-gated chloride channel activity [GO:0061797], serotonin-gated chloride channel activity [GO:0160039] Sources: GOC:mtg_transport, ISBN:0815340729 Relationships: is a type of monoatomic anion channel activity [GO:0005253]; is a type of ligand-gated monoatomic ion channel activity [GO:0015276]